{
  "term_id": "UNKNOWN:0001",
  "gene": "UniProtKB:Q96NC0",
  "gene_name": "Zinc finger matrin-type protein 2",
  "gene_symbol": "ZMAT2",
  "term_label": "Unknown molecular function"
}